{
  "gene_name": "Dynamin-1-like protein",
  "gene_symbol": "DNM1L",
  "gene": "UniProtKB:O00429",
  "term_label": "intracellular distribution of mitochondria",
  "term_id": "GO:0048312"
}